{
  "term_id": "GO:0016324",
  "gene_name": "Na(+)_H(+) exchange regulatory cofactor NHE-RF3",
  "term_label": "apical plasma membrane",
  "gene": "UniProtKB:Q5T2W1",
  "gene_symbol": "PDZK1"
}